{
  "gene_symbol": "PSMC6",
  "term_label": "proteasome-mediated ubiquitin-dependent protein catabolic process",
  "gene_name": "26S proteasome regulatory subunit 10B",
  "gene": "UniProtKB:P62333",
  "term_id": "GO:0043161"
}